regulation of calcium import into the mitochondrion [GO:0110097] (biological process) Definition: Any process that modulates the frequency, rate or extent of calcium import into the mitochondrion. References: PMID:24085037 Sources: GOC:sl Subtypes: positive regulation of calcium import into the mitochondrion [GO:0110098], negative regulation of calcium import into the mitochondrion [GO:0110099] Relationships: is a type of GO:1903169; regulates calcium import into the mitochondrion [GO:0036444]